{
  "gene_name": "Serine_threonine-protein kinase 26",
  "term_id": "GO:0035556",
  "gene": "UniProtKB:Q9P289",
  "term_label": "intracellular signal transduction",
  "gene_symbol": "STK26"
}